branchiomotor neuron axon guidance in neural tube [GO:0021786] (BP) Relationships: is a type of branchiomotor neuron axon guidance [GO:0021785] References: PMID:14699587 Sources: GOC:cls, GOC:dgh, GOC:dph, GOC:jid, GO_REF:0000021 Subtypes: chemorepulsion of branchiomotor neuron axon in neural tube [GO:0021787], chemoattraction of branchiomotor neuron axon in neural tube [GO:0021788] Definition: The process in which a branchiomotor neuron growth cone in the neural tube is directed to a specific target site in the neural tube. Branchiomotor neurons are located in the hindbrain and innervate branchial arch-derived muscles that control jaw movements, facial expression, the larynx, and the pharynx.